{
  "gene_symbol": "SH2D4B",
  "term_label": "protein-macromolecule adaptor activity",
  "gene_name": "SH2 domain-containing protein 4B",
  "term_id": "GO:0030674",
  "gene": "UniProtKB:Q5SQS7"
}